{
  "gene_symbol": "FAM220A",
  "gene": "UniProtKB:Q7Z4H9",
  "gene_name": "Protein FAM220A",
  "term_id": "UNKNOWN:0002",
  "term_label": "Unknown biological process"
}